retrograde trans-synaptic signaling by nitric oxide [GO:0098924] (biological process) Definition: Cell-cell signaling from postsynapse to presynapse, across the synaptic cleft, mediated by nitric oxide. Subtypes: GO:0098925 Relationships: is a type of retrograde trans-synaptic signaling by soluble gas [GO:0098923]; is a type of trans-synaptic signaling by nitric oxide [GO:0099548] Sources: GOC:dos